acidic amino acid transmembrane transporter activity [GO:0015172] (molecular function) Definition: Enables the transfer of acidic amino acids from one side of a membrane to the other. Acidic amino acids have side chains with a negative charge at pH 7.3. Subtypes: L-glutamate transmembrane transporter activity [GO:0005313], L-aspartate transmembrane transporter activity [GO:0015183] Relationships: is_a amino acid transmembrane transporter activity [GO:0015171]; is part of acidic amino acid transport [GO:0015800] Sources: GOC:ai, GOC:mtg_transport, ISBN:0815340729 Also known as: acidic amino acid transporter activity